{
  "term_id": "GO:0004745",
  "gene": "UniProtKB:Q9NYR8",
  "gene_symbol": "RDH8",
  "gene_name": "Retinol dehydrogenase 8",
  "term_label": "all-trans-retinol dehydrogenase (NAD+) activity"
}